regulation of hypersensitivity [GO:0002883] (biological process) Definition: Any process that modulates the frequency, rate, or extent of hypersensitivity. Relationships: is a type of regulation of acute inflammatory response to antigenic stimulus [GO:0002864]; regulates hypersensitivity [GO:0002524] Sources: GOC:add Subtypes: regulation of type III hypersensitivity [GO:0001803], regulation of type IV hypersensitivity [GO:0001807], regulation of type I hypersensitivity [GO:0001810], negative regulation of hypersensitivity [GO:0002884], positive regulation of hypersensitivity [GO:0002885], regulation of type II hypersensitivity [GO:0002892]